{
  "gene_symbol": "PIM2",
  "gene": "UniProtKB:Q9P1W9",
  "term_id": "GO:0004674",
  "gene_name": "Serine_threonine-protein kinase pim-2",
  "term_label": "protein serine/threonine kinase activity"
}